{
  "term_id": "GO:0005634",
  "term_label": "nucleus",
  "gene_symbol": "LGALS3",
  "gene_name": "Galectin-3",
  "gene": "UniProtKB:P17931"
}